{
  "term_id": "UNKNOWN:0003",
  "gene_name": "Immunoglobulin heavy variable 3_OR16-17 (non-functional) (Fragment)",
  "gene_symbol": "IGHV3OR16-17",
  "term_label": "Unknown cellular component",
  "gene": "UniProtKB:S4R3C0"
}